{
  "gene_name": "Sentan",
  "gene_symbol": "SNTN",
  "term_label": "Unknown cellular component",
  "gene": "UniProtKB:A6NMZ2",
  "term_id": "UNKNOWN:0003"
}